{
  "term_label": "regulation of transcription by RNA polymerase II",
  "gene": "UniProtKB:Q9UC07",
  "gene_name": "Zinc finger protein 69",
  "term_id": "GO:0006357",
  "gene_symbol": "ZNF69"
}